{
  "gene_name": "SIGLEC family-like protein 1",
  "term_id": "UNKNOWN:0001",
  "gene": "UniProtKB:Q8N7X8",
  "term_label": "Unknown molecular function",
  "gene_symbol": "SIGLECL1"
}